definitive erythrocyte differentiation [GO:0060318] (BP) Relationships: is a type of erythrocyte differentiation [GO:0030218]; is part of GO:0060216 Sources: GOC:BHF, GOC:add, GOC:dph Regulation: regulated by regulation of definitive erythrocyte differentiation [GO:0010724] Definition: Erythrocyte differentiation which occurs as part of the process of definitive hemopoiesis. Also known as: definitive RBC differentiation, definitive erythropoiesis, definitive red blood cell differentiation